{
  "gene_name": "Olfactory receptor 8U8",
  "gene_symbol": "OR8U8",
  "gene": "UniProtKB:P0C7N1",
  "term_id": "UNKNOWN:0001",
  "term_label": "Unknown molecular function"
}